{
  "term_id": "GO:0010369",
  "gene_name": "Methyl-CpG-binding domain protein 6",
  "gene_symbol": "MBD6",
  "term_label": "chromocenter",
  "gene": "UniProtKB:Q96DN6"
}